regulation of hematopoietic progenitor cell differentiation [GO:1901532] (biological process) Subtypes: negative regulation of hematopoietic progenitor cell differentiation [GO:1901533], GO:1901534, regulation of hematopoietic stem cell differentiation [GO:1902036], regulation of myeloid progenitor cell differentiation [GO:1905453], regulation of lymphoid progenitor cell differentiation [GO:1905456] Also known as: regulation of haematopoietic progenitor cell differentiation, regulation of haemopoietic progenitor cell differentiation, regulation of hemopoietic progenitor cell differentiation Definition: Any process that modulates the frequency, rate or extent of hematopoietic progenitor cell differentiation. Sources: GOC:BHF, GOC:TermGenie, GOC:rl Relationships: is a type of GO:0045595; regulates GO:0002244